{
  "term_id": "GO:0008270",
  "gene_name": "Nuclear transition protein 2",
  "gene": "UniProtKB:Q05952",
  "gene_symbol": "TNP2",
  "term_label": "zinc ion binding"
}